L-cystine reductase (NADH) activity [GO:0050456] (molecular function) Definition: Catalysis of the reaction: 2 L-cysteine + NAD+ = L-cystine + H+ + NADH. Also known as: cystine reductase activity, L-cysteine:NAD+ oxidoreductase, NADH-dependent cystine reductase activity, NADH2:L-cystine oxidoreductase, NADH:L-cystine oxidoreductase activity, cystine reductase (NADH) activity, cystine reductase (NADH2) Relationships: is a type of oxidoreductase activity, acting on a sulfur group of donors, NAD(P) as acceptor [GO:0016668] Sources: EC:1.8.1.6, RHEA:20597